{
  "gene_symbol": "CDH11",
  "gene_name": "Cadherin-11",
  "gene": "UniProtKB:P55287",
  "term_label": "cell morphogenesis",
  "term_id": "GO:0000902"
}